{
  "gene_name": "Putative glycine N-acyltransferase-like protein 1B",
  "gene_symbol": "GLYATL1B",
  "gene": "UniProtKB:A0A0U1RQE8",
  "term_id": "GO:0006541",
  "term_label": "glutamine metabolic process"
}